{
  "gene_name": "Putative apolipoprotein(a)-like protein 2",
  "term_id": "UNKNOWN:0001",
  "term_label": "Unknown molecular function",
  "gene_symbol": "LPAL2",
  "gene": "UniProtKB:Q16609"
}